vasopressin secretion [GO:0030103] (biological process) Sources: GOC:mah Relationships: is_a peptide hormone secretion [GO:0030072] Subtypes: secretion of vasopressin involved in fast regulation of systemic arterial blood pressure [GO:0002004] Definition: The regulated release of vasopressin from secretory granules into the blood.